{
  "gene_symbol": "GARIN4",
  "gene": "UniProtKB:Q8IYT1",
  "term_id": "UNKNOWN:0003",
  "gene_name": "Golgi-associated RAB2 interactor protein 4",
  "term_label": "Unknown cellular component"
}